{
  "term_id": "GO:0098982",
  "gene": "UniProtKB:Q96NI6",
  "gene_symbol": "LRFN5",
  "gene_name": "Leucine-rich repeat and fibronectin type-III domain-containing protein 5",
  "term_label": "GABA-ergic synapse"
}